{
  "gene_name": "Olfactory receptor 4C13",
  "term_id": "GO:0005886",
  "gene_symbol": "OR4C13",
  "term_label": "plasma membrane",
  "gene": "UniProtKB:Q8NGP0"
}